{
  "gene_name": "PRAME family member 14",
  "gene_symbol": "PRAMEF14",
  "term_label": "Cul2-RING ubiquitin ligase complex",
  "gene": "UniProtKB:Q5SWL7",
  "term_id": "GO:0031462"
}